regulation of type III hypersensitivity [GO:0001803] (biological process) Subtypes: GO:0001804, positive regulation of type III hypersensitivity [GO:0001805] Definition: Any process that modulates the frequency, rate, or extent of type III hypersensitivity, a type of inflammatory response. Relationships: is a type of regulation of hypersensitivity [GO:0002883]; is a type of GO:0002886; is a type of regulation of immunoglobulin mediated immune response [GO:0002889]; regulates type III hypersensitivity [GO:0001802] Sources: GOC:add, ISBN:0781735149